{
  "gene": "UniProtKB:Q9UH03",
  "term_label": "cell division site",
  "term_id": "GO:0032153",
  "gene_name": "Neuronal-specific septin-3",
  "gene_symbol": "SEPTIN3"
}